{
  "gene": "UniProtKB:Q9NR77",
  "gene_name": "Peroxisomal membrane protein 2",
  "term_id": "GO:0005737",
  "gene_symbol": "PXMP2",
  "term_label": "cytoplasm"
}